{
  "gene": "UniProtKB:Q7Z6G3",
  "term_label": "cytoplasm",
  "term_id": "GO:0005737",
  "gene_symbol": "NECAB2",
  "gene_name": "N-terminal EF-hand calcium-binding protein 2"
}